{
  "gene_symbol": "IL10",
  "term_id": "GO:0005125",
  "gene": "UniProtKB:P22301",
  "gene_name": "Interleukin-10",
  "term_label": "cytokine activity"
}